cytochrome b6f complex [GO:0009512] (cellular component) Definition: Complex that transfers electrons from reduced plastoquinone to oxidized plastocyanin and translocates protons from the stroma to the lumen. The complex contains a core structure of three catalytic subunits: cytochrome b, the Rieske iron sulfur protein (ISP), and cytochrome f, which are arranged in an integral membrane-bound dimeric complex; additional subunits are present, and vary among different species. Also known as: cyt b(6)f complex, cyt b6-f complex, cyt b6/f complex, cyt b6f complex, cytochrome b(6)f complex, cytochrome b6-f complex, cytochrome b6/f complex Relationships: is a type of cytochrome complex [GO:0070069]; is part of GO:0009579 References: PMID:16228398, PMID:16352458 Sources: ISBN:0943088399